{
  "term_id": "GO:0005739",
  "gene": "UniProtKB:Q8NI37",
  "term_label": "mitochondrion",
  "gene_name": "Protein phosphatase PTC7 homolog",
  "gene_symbol": "PPTC7"
}